{
  "gene_name": "Mitogen-activated protein kinase kinase kinase 19",
  "term_id": "GO:0000165",
  "gene_symbol": "MAP3K19",
  "gene": "UniProtKB:Q56UN5",
  "term_label": "MAPK cascade"
}